adenylate cyclase inhibiting G protein-coupled glutamate receptor activity [GO:0001640] (molecular function) Also known as: adenylyl cyclase inhibiting metabotropic glutamate receptor activity, adenylate cyclase inhibiting metabotropic glutamate receptor activity Definition: Combining with glutamate and transmitting the signal across the membrane by activating the alpha-subunit of an associated heterotrimeric G-protein complex to inhibit downstream adenylate cyclase activity. Relationships: is a type of GO:0098988; is part of adenylate cyclase-inhibiting G protein-coupled glutamate receptor signaling pathway [GO:0007196] Subtypes: GO:0001641, GO:0001642 Sources: GOC:bf, GOC:dph